{
  "term_label": "neutral amino acid transport",
  "gene_name": "Large neutral amino acids transporter small subunit 4",
  "gene": "UniProtKB:Q8N370",
  "gene_symbol": "SLC43A2",
  "term_id": "GO:0015804"
}